bombesin receptor signaling pathway [GO:0031989] (biological process) Definition: A G protein-coupled receptor signaling pathway initiated by a bombesin binding to its receptor, and ending with the regulation of a downstream cellular process, e.g. transcription. Sources: GOC:mah Also known as: bombesin receptor signalling pathway Relationships: is a type of GO:0007186